{
  "gene_name": "Actin remodeling regulator NHS",
  "term_id": "UNKNOWN:0001",
  "term_label": "Unknown molecular function",
  "gene": "UniProtKB:Q6T4R5",
  "gene_symbol": "NHS"
}